{
  "gene_symbol": "TIMM17A",
  "gene_name": "Mitochondrial import inner membrane translocase subunit Tim17-A",
  "gene": "UniProtKB:Q99595",
  "term_id": "GO:0030150",
  "term_label": "protein import into mitochondrial matrix"
}